{
  "gene_symbol": "ISOC2",
  "gene_name": "Isochorismatase domain-containing protein 2",
  "gene": "UniProtKB:Q96AB3",
  "term_id": "UNKNOWN:0002",
  "term_label": "Unknown biological process"
}